{
  "gene": "UniProtKB:Q6QAJ8",
  "gene_symbol": "TMEM220",
  "gene_name": "Transmembrane protein 220",
  "term_label": "Unknown biological process",
  "term_id": "UNKNOWN:0002"
}